{
  "term_id": "GO:0005876",
  "gene_name": "Aurora kinase C",
  "term_label": "spindle microtubule",
  "gene": "UniProtKB:Q9UQB9",
  "gene_symbol": "AURKC"
}